curcumin reductase (NADP+) activity [GO:0052849] (molecular function) Sources: RHEA:34815 Also known as: NADPH-dependent curcumin reductase activity Definition: Catalysis of the reaction: 2 NADP+ + tetrahydrocurcumin = curcumin + 2 H+ + 2 NADPH. Relationships: is a type of oxidoreductase activity, acting on the CH-CH group of donors, NAD or NADP as acceptor [GO:0016628]